reuteran biosynthetic process [GO:0052784] (biological process) Also known as: reuteransucrase-mediated reuteran biosynthesis Definition: The chemical reactions and pathways resulting in the formation of reuteran, a soluble glucan polymer with mainly alpha-(1->4) glycosidic linkages and significant amounts of alpha-(1->6) and alpha-(1->4,6) glucosidic linkages. References: PMID:15256553, PMID:16000808 Sources: GOC:mengo_curators Relationships: is a type of alpha-glucan biosynthetic process [GO:0030979]